regulation of gluconate transmembrane transport [GO:0035430] (biological process) Definition: Any process that modulates the frequency, rate or extent of the directed movement of a gluconate across a membrane by means of some agent such as a transporter or pore. Sources: GOC:vw Also known as: regulation of gluconate membrane transport, regulation of gluconate transport Relationships: is a type of regulation of organic acid transport [GO:0032890]; is a type of regulation of transmembrane transport [GO:0034762]; regulates gluconate transmembrane transport [GO:0035429] Subtypes: GO:0035431, positive regulation of gluconate transmembrane transport [GO:0035432]